{
  "gene": "UniProtKB:Q14943",
  "gene_symbol": "KIR3DS1",
  "term_label": "immune response-inhibiting cell surface receptor signaling pathway",
  "term_id": "GO:0002767",
  "gene_name": "Killer cell immunoglobulin-like receptor 3DS1"
}